anterior lateral line nerve glial cell morphogenesis involved in differentiation [GO:0048940] (biological process) Sources: GOC:dgh Definition: The process in which the structures of a glial cell in the anterior lateral line nerve are generated and organized. This process occurs while the initially relatively unspecialized cell is acquiring the specialized features of a glial cell in the anterior lateral line nerve. Relationships: is_a lateral line nerve glial cell morphogenesis involved in differentiation [GO:0048938]; is part of anterior lateral line nerve glial cell development [GO:0048939]